cellular response to vitamin E [GO:0071306] (biological process) Also known as: cellular response to DL-alpha-tocopherol acetate, cellular response to DL-alpha-tocopheryl acetate, cellular response to O-Acetyl-alpha-tocopherol Definition: Any process that results in a change in state or activity of a cell (in terms of movement, secretion, enzyme production, gene expression, etc.) as a result of a vitamin E stimulus. Sources: GOC:mah Relationships: is a type of response to vitamin E [GO:0033197]; is_a cellular response to vitamin [GO:0071295]; is a type of cellular response to oxygen-containing compound [GO:1901701]